glucose-1-phosphate phosphodismutase activity [GO:0047937] (MF) Relationships: is a type of kinase activity [GO:0016301]; is_a phosphotransferase activity, alcohol group as acceptor [GO:0016773] Sources: EC:2.7.1.41, MetaCyc:GLUCOSE-1-PHOSPHATE-PHOSPHODISMUTASE-RXN Definition: Catalysis of the reaction: 2 D-glucose 1-phosphate = D-glucose + D-glucose 1,6-bisphosphate. Also known as: D-glucose-1-phosphate:D-glucose-1-phosphate 6-phosphotransferase activity, glucose 1-phosphate transphosphorylase activity, phosphodismutase activity